{
  "term_id": "GO:0000278",
  "term_label": "mitotic cell cycle",
  "gene_symbol": "TUBB2A",
  "gene": "UniProtKB:Q13885",
  "gene_name": "Tubulin beta-2A chain"
}